{
  "term_label": "Unknown molecular function",
  "term_id": "UNKNOWN:0001",
  "gene_symbol": "LRRC18",
  "gene": "UniProtKB:Q8N456",
  "gene_name": "Leucine-rich repeat-containing protein 18"
}